{
  "gene_name": "NADH dehydrogenase [ubiquinone] 1 alpha subcomplex subunit 3",
  "term_label": "Unknown biological process",
  "gene_symbol": "NDUFA3",
  "term_id": "UNKNOWN:0002",
  "gene": "UniProtKB:O95167"
}